aldose 1-dehydrogenase activity [GO:0047640] (molecular function) Definition: Catalysis of the reaction: D-aldose + NAD+ = D-aldonolactone + NADH. Sources: EC:1.1.1.121, MetaCyc:ALDOSE-1-DEHYDROGENASE-RXN Relationships: is a type of oxidoreductase activity, acting on the CH-OH group of donors, NAD or NADP as acceptor [GO:0016616] Also known as: D-aldose:NAD+ 1-oxidoreductase activity, aldose dehydrogenase activity, dehydrogenase, D-aldohexose